{
  "term_label": "Unknown cellular component",
  "term_id": "UNKNOWN:0003",
  "gene_symbol": "TROAP",
  "gene_name": "Tastin",
  "gene": "UniProtKB:Q12815"
}